{
  "gene": "UniProtKB:Q9UKJ0",
  "term_label": "Unknown biological process",
  "gene_symbol": "PILRB",
  "term_id": "UNKNOWN:0002",
  "gene_name": "Paired immunoglobulin-like type 2 receptor beta"
}